{
  "term_label": "DNA binding",
  "term_id": "GO:0003677",
  "gene_symbol": "H2BK1",
  "gene": "UniProtKB:A0A2R8Y619",
  "gene_name": "Histone H2B type 2-K1"
}